{
  "gene_name": "Tetratricopeptide repeat protein 23-like",
  "gene_symbol": "TTC23L",
  "term_label": "Unknown molecular function",
  "term_id": "UNKNOWN:0001",
  "gene": "UniProtKB:Q6PF05"
}